{
  "term_id": "GO:0004879",
  "gene_name": "Retinoic acid receptor RXR-gamma",
  "gene": "UniProtKB:P48443",
  "term_label": "nuclear receptor activity",
  "gene_symbol": "RXRG"
}